{
  "gene_name": "Transmembrane and immunoglobulin domain-containing protein 2",
  "gene_symbol": "TMIGD2",
  "term_id": "GO:0043005",
  "gene": "UniProtKB:Q96BF3",
  "term_label": "neuron projection"
}